prenylcysteine oxidase activity [GO:0001735] (molecular function) Definition: Catalysis of the reaction: S-prenyl-L-cysteine + O2 + H2O = a prenal + L-cysteine + H2O2. Sources: GOC:hjd, RHEA:53892 Also known as: S-prenyl-L-cysteine:oxygen oxidoreductase activity, prenylcysteine lyase activity Relationships: is a type of oxidoreductase activity, acting on a sulfur group of donors, oxygen as acceptor [GO:0016670]